{
  "term_id": "GO:0009617",
  "gene_symbol": "TRAV4",
  "term_label": "response to bacterium",
  "gene_name": "T cell receptor alpha variable 4",
  "gene": "UniProtKB:A0A0B4J268"
}